asparagusate reductase (NADH) activity [GO:0050445] (molecular function) Relationships: is a type of oxidoreductase activity, acting on a sulfur group of donors, NAD(P) as acceptor [GO:0016668] Definition: Catalysis of the reaction: 3-sulfanyl-2-(sulfanylmethyl)propanoate + NAD+ = asparagusate + NADH + H+. Sources: RHEA:14881 Also known as: asparagusate reductase activity, 3-mercapto-2-mercaptomethylpropanoate:NAD+ oxidoreductase activity, NADH2:asparagusate oxidoreductase activity, NADH:asparagusate oxidoreductase activity, asparagusate dehydrogenase activity, asparagusate reductase (NADH2), asparagusic dehydrogenase activity